{
  "gene_name": "Methylosome subunit pICln",
  "term_label": "spliceosomal snRNP assembly",
  "gene": "UniProtKB:P54105",
  "term_id": "GO:0000387",
  "gene_symbol": "CLNS1A"
}